respiratory burst after phagocytosis [GO:0045728] (biological process) Definition: A phase of elevated metabolic activity, during which oxygen consumption increases, that occurs in neutrophils, monocytes, and macrophages shortly after phagocytosing material. An enhanced uptake of oxygen leads to the production, by an NADH dependent system, of hydrogen peroxide (H2O2), superoxide anions and hydroxyl radicals, which play a part in microbiocidal activity. Sources: GOC:curators, ISBN:0198506732 Also known as: metabolic burst after phagocytosis, oxidative burst after phagocytosis Relationships: is a type of respiratory burst involved in defense response [GO:0002679]